{
  "gene_name": "Serine_threonine-protein kinase LMTK3",
  "gene_symbol": "LMTK3",
  "term_label": "protein kinase activity",
  "term_id": "GO:0004672",
  "gene": "UniProtKB:Q96Q04"
}